bHLH transcription factor binding [GO:0043425] (molecular function) References: PMID:9144210 Subtypes: MRF binding [GO:0043426] Relationships: is a type of DNA-binding transcription factor binding [GO:0140297] Definition: Binding to a basic Helix-Loop-Helix (bHLH) superfamily of transcription factors, important regulatory components in transcriptional networks of many developmental pathways.